{
  "gene_name": "Methenyltetrahydrofolate synthase domain-containing protein",
  "term_label": "Unknown biological process",
  "gene": "UniProtKB:Q2M296",
  "gene_symbol": "MTHFSD",
  "term_id": "UNKNOWN:0002"
}